{
  "term_id": "GO:0000978",
  "gene_name": "Nuclear factor of activated T-cells, cytoplasmic 3",
  "gene": "UniProtKB:Q12968",
  "gene_symbol": "NFATC3",
  "term_label": "RNA polymerase II cis-regulatory region sequence-specific DNA binding"
}